{
  "gene_name": "Cilia- and flagella-associated protein 77",
  "gene": "UniProtKB:Q6ZQR2",
  "gene_symbol": "CFAP77",
  "term_id": "UNKNOWN:0003",
  "term_label": "Unknown cellular component"
}